regulation of capsule polysaccharide biosynthetic process [GO:0062084] (biological process) Subtypes: positive regulation of capsule polysaccharide biosynthetic process [GO:0062085] Definition: Any process that modulates the frequency, rate or extent of the chemical reactions and pathways resulting in the formation of polysaccharides that make up the capsule, a protective structure surrounding some species of bacteria and fungi. Relationships: is a type of regulation of polysaccharide biosynthetic process [GO:0032885]; is a type of regulation of capsule organization [GO:1901913]; regulates capsule polysaccharide biosynthetic process [GO:0045227] References: PMID:21917918